methylselenol demethylase activity [GO:0098608] (molecular function) Definition: Catalysis of the reaction: methylselenol + H2O = H2Se + CH3OH. Relationships: is a type of demethylase activity [GO:0032451] References: PMID:17451884, PMID:17988700